{
  "term_label": "carnosine metabolic process",
  "gene": "UniProtKB:Q8N4J0",
  "gene_symbol": "CARNMT1",
  "gene_name": "Carnosine N-methyltransferase",
  "term_id": "GO:0035498"
}